renal vesicle formation [GO:0072033] (BP) Definition: The developmental process pertaining to the initial formation of the renal vesicle from condensed mesenchymal cells. The renal vesicle is the primordial structure of the nephron epithelium, and is formed by the condensation of mesenchymal cells. Relationships: is_a GO:0048646; is part of GO:0072077 Sources: GOC:mtg_kidney_jan10 Subtypes: mesonephric renal vesicle formation [GO:0061262], metanephric renal vesicle formation [GO:0072093] Also known as: nephron epithelium formation Regulation: positively regulated by renal vesicle induction [GO:0072034]